{
  "gene": "UniProtKB:Q96KT6",
  "term_label": "Unknown molecular function",
  "term_id": "UNKNOWN:0001",
  "gene_name": "Putative uncharacterized protein encoded by LINC00208",
  "gene_symbol": "LINC00208"
}